negative regulation of cartilage condensation [GO:1904932] (biological process) References: PMID:17604018 Sources: GOC:TermGenie, GOC:mr, GO_REF:0000058 Definition: Any process that stops, prevents or reduces the frequency, rate or extent of cartilage condensation. Also known as: down regulation of cartilage condensation, down-regulation of cartilage condensation, downregulation of cartilage condensation, inhibition of cartilage condensation Relationships: is a type of negative regulation of cellular process [GO:0048523]; is a type of regulation of cartilage condensation [GO:1902026]; negatively regulates cartilage condensation [GO:0001502]